{
  "term_id": "GO:0001222",
  "gene_symbol": "PER2",
  "term_label": "transcription corepressor binding",
  "gene": "UniProtKB:O15055",
  "gene_name": "Period circadian protein homolog 2"
}